{
  "term_id": "GO:0030574",
  "term_label": "collagen catabolic process",
  "gene_symbol": "MMP13",
  "gene": "UniProtKB:P45452",
  "gene_name": "Collagenase 3"
}